{
  "gene_symbol": "PLCL1",
  "gene_name": "Inactive phospholipase C-like protein 1",
  "term_id": "GO:0007214",
  "term_label": "gamma-aminobutyric acid signaling pathway",
  "gene": "UniProtKB:Q15111"
}